axonemal dynein complex assembly [GO:0070286] (biological process) Subtypes: outer dynein arm assembly [GO:0036158], inner dynein arm assembly [GO:0036159] Relationships: is a type of GO:0065003; is part of axoneme assembly [GO:0035082] Definition: The aggregation, arrangement and bonding together of a set of components to form an axonemal dynein complex, a dynein complex found in eukaryotic cilia and flagella, in which the motor domain heads interact with adjacent microtubules to generate a sliding force which is converted to a bending motion. References: PMID:19052621 Sources: GOC:cilia, GOC:mah Also known as: dynein arm assembly